{
  "term_label": "ATP transport",
  "gene": "UniProtKB:Q9BV35",
  "gene_name": "Mitochondrial adenyl nucleotide antiporter SLC25A23",
  "term_id": "GO:0015867",
  "gene_symbol": "SLC25A23"
}